floppase activity [GO:0140328] (molecular function) Definition: Catalysis of the movement of a lipid from the cytosolic to the exoplasmic leaflet of a membrane, using energy from the hydrolysis of ATP. Note: Nomenclature note. Flippases and floppases are ATP-dependent transbilayer lipid translocators. According to an extensively used, though not universal, nomenclature, they catalyze lipid transfer towards the inward monolayer (flippases) or towards the outward monolayer (floppases). Scramblases are ATP-independent, non-selective, inducing non-specific transbilayer movements across the membrane. The direction of the translocation should be taken into account for annotation (from the cytosolic to the exoplasmic leaflet of a membrane). Also known as: floppase activity (cytosolic to exoplasmic leaflet) Subtypes: GO:0015161, GO:0015437, glycolipid floppase activity [GO:0034202], GO:0046623, phosphatidylcholine floppase activity [GO:0090554], phosphatidylserine floppase activity [GO:0090556], phosphatidylethanolamine floppase activity [GO:0140341] Relationships: is a type of ATPase-coupled intramembrane lipid transporter activity [GO:0140326] References: PMID:20043909, PMID:25284293 Sources: Wikipedia:Flippase